actomyosin contractile ring organization [GO:0044837] (biological process) Sources: GOC:mtg_cell_cycle Also known as: cytokinesis, actomyosin contractile ring organization Relationships: is a type of GO:0022402; is a type of cortical actin cytoskeleton organization [GO:0030866]; is_a actomyosin structure organization [GO:0031032]; is part of cytoskeleton-dependent cytokinesis [GO:0061640] Definition: A process which results in the assembly, arrangement of constituent parts, or disassembly of an actomyosin contractile ring. Subtypes: actomyosin contractile ring assembly [GO:0000915], actomyosin contractile ring maturation [GO:0031566]